negative regulation of substrate adhesion-dependent cell spreading [GO:1900025] (biological process) Also known as: down regulation of cell spreading during cell substrate adhesion, down regulation of substrate adhesion dependent cell spreading, negative regulation of cell spreading during cell substrate adhesion, negative regulation of substrate adhesion dependent cell spreading, down regulation of substrate adhesion-dependent cell spreading Definition: Any process that stops, prevents or reduces the frequency, rate or extent of substrate adhesion-dependent cell spreading. Relationships: is a type of negative regulation of cell-substrate adhesion [GO:0010812]; is a type of GO:1900024; negatively regulates substrate adhesion-dependent cell spreading [GO:0034446] Sources: GOC:TermGenie, GOC:yaf